kynurenine metabolic process [GO:0070189] (biological process) Also known as: kynurenine metabolism Relationships: is a type of ketone metabolic process [GO:0042180]; is a type of benzene-containing compound metabolic process [GO:0042537]; is a type of GO:0170041; is a type of alpha-amino acid metabolic process [GO:1901605] Subtypes: L-tryptophan catabolic process to kynurenine [GO:0019441], L-kynurenine metabolic process [GO:0097052] Sources: CHEBI:28683, GOC:mah, GOC:rph Definition: The chemical reactions and pathways involving kynurenine, the amino acid 3-(2-aminobenzoyl)-alanine.